{
  "term_id": "UNKNOWN:0002",
  "gene_symbol": "Q9BRP9",
  "gene": "UniProtKB:Q9BRP9",
  "term_label": "Unknown biological process",
  "gene_name": "Putative uncharacterized protein MGC13053"
}